methyltransferase cap1 activity [GO:0004483] (molecular function) Sources: EC:2.1.1.57 Definition: Catalysis of the reaction: a 5'-end (N(7)-methyl 5'-triphosphoguanosine)-ribonucleoside in mRNA or snRNA + S-adenosyl-L-methionine = a 5'-end (N(7)-methyl 5'-triphosphoguanosine)-(2'-O-methyl-ribonucleoside) in mRNA or snRNA + S-adenosyl-L-homocysteine + H+. This activity catalyzes the methylation of the ribose on the first transcribed nucleotide of mRNAs and snRNAs. Relationships: is a type of O-methyltransferase activity [GO:0008171]; is a type of RNA methyltransferase activity [GO:0008173] Also known as: S-adenosyl-L-methionine:mRNA (nucleoside-2'-O-)-methyltransferase activity, mRNA (adenosine-2'-O-)-methyltransferase activity, mRNA (nucleoside-2'-O-)-methyltransferase activity, messenger RNA (nucleoside-2'-)-methyltransferase activity, messenger ribonucleate nucleoside 2'-methyltransferase activity